{
  "gene_symbol": "C1orf53",
  "gene_name": "Uncharacterized protein C1orf53",
  "gene": "UniProtKB:Q5VUE5",
  "term_id": "UNKNOWN:0002",
  "term_label": "Unknown biological process"
}